regulation of cellular response to vascular endothelial growth factor stimulus [GO:1902547] (biological process) Relationships: is a type of GO:0090287; regulates cellular response to vascular endothelial growth factor stimulus [GO:0035924] Definition: Any process that modulates the frequency, rate or extent of cellular response to vascular endothelial growth factor stimulus. Also known as: regulation of cellular response to VEGF, regulation of cellular response to vascular endothelial growth factor, regulation of cellular response to VEGFA, regulation of cellular response to VEGFB Subtypes: regulation of vascular endothelial growth factor signaling pathway [GO:1900746], negative regulation of cellular response to vascular endothelial growth factor stimulus [GO:1902548], regulation of endothelial cell chemotaxis to vascular endothelial growth factor [GO:1904857] References: PMID:17895370 Sources: GOC:BHF, GOC:TermGenie, GOC:rl